{
  "gene_name": "Protein monoglycylase TTLL8",
  "gene_symbol": "TTLL8",
  "term_label": "axoneme",
  "gene": "UniProtKB:A6PVC2",
  "term_id": "GO:0005930"
}